{
  "term_id": "GO:0005737",
  "term_label": "cytoplasm",
  "gene_name": "Serine_threonine-protein phosphatase 2B catalytic subunit beta isoform",
  "gene": "UniProtKB:P16298",
  "gene_symbol": "PPP3CB"
}